{
  "gene": "UniProtKB:Q86W11",
  "term_label": "RNA polymerase II cis-regulatory region sequence-specific DNA binding",
  "term_id": "GO:0000978",
  "gene_symbol": "ZSCAN30",
  "gene_name": "Zinc finger and SCAN domain-containing protein 30"
}